{
  "gene": "UniProtKB:P02795",
  "gene_symbol": "MT2A",
  "gene_name": "Metallothionein-2",
  "term_label": "nucleus",
  "term_id": "GO:0005634"
}